{
  "gene_symbol": "GAP43",
  "term_id": "GO:0005516",
  "gene": "UniProtKB:P17677",
  "term_label": "calmodulin binding",
  "gene_name": "Neuromodulin"
}